{
  "gene": "UniProtKB:A0A1B0GWB2",
  "term_id": "GO:0016020",
  "gene_symbol": "PRRT1B",
  "term_label": "membrane",
  "gene_name": "Proline rich transmembrane protein 1B"
}